pyridoxal binding [GO:0070280] (molecular function) Sources: CHEBI:17310, GOC:mah Relationships: is a type of cation binding [GO:0043169]; is a type of GO:0070279 Definition: Binding to pyridoxal, 3-hydroxy-5-(hydroxymethyl)-2-methylpyridine-4-carbaldehyde, a form of vitamin B6.